{
  "term_id": "GO:0070761",
  "term_label": "pre-snoRNP complex",
  "gene_name": "Box C_D snoRNA protein 1",
  "gene_symbol": "ZNHIT6",
  "gene": "UniProtKB:Q9NWK9"
}